{
  "gene": "UniProtKB:A0A0B4J1Y8",
  "gene_name": "Immunoglobulin lambda variable 9-49",
  "term_label": "Unknown molecular function",
  "gene_symbol": "IGLV9-49",
  "term_id": "UNKNOWN:0001"
}